interphase mitotic telomere clustering [GO:0120110] (biological process) Note: It is likely that both intra chromosome telomere clustering and inter-chromosome occur because a single focus is sometimes observed, although this has yet to be proven. Definition: The process whereby the mitotic telomeres are gathered together during, or prior to, attachment to the nuclear envelope. Relationships: is a type of telomere localization [GO:0034397]; is part of mitotic telomere clustering and tethering at nuclear periphery [GO:0120109] Also known as: mitotic telomere clustering during interphase Regulation: regulated by GO:0110065; negatively regulated by negative regulation of interphase mitotic telomere clustering [GO:0110066] References: PMID:25778919